{
  "gene": "UniProtKB:O76009",
  "term_id": "GO:0030855",
  "term_label": "epithelial cell differentiation",
  "gene_symbol": "KRT33A",
  "gene_name": "Keratin, type I cuticular Ha3-I"
}